mitochondrial ribosome [GO:0005761] (cellular component) Definition: A ribosome found in the mitochondrion of a eukaryotic cell; contains a characteristic set of proteins distinct from those of cytosolic ribosomes. Sources: GOC:mah, ISBN:0198506732 Also known as: 55S ribosome, mitochondrial Relationships: is a type of organellar ribosome [GO:0000313]; is part of mitochondrial matrix [GO:0005759]